{
  "gene_symbol": "WDR45B",
  "gene_name": "WD repeat domain phosphoinositide-interacting protein 3",
  "gene": "UniProtKB:Q5MNZ6",
  "term_label": "cytosol",
  "term_id": "GO:0005829"
}